{
  "term_label": "plasma membrane",
  "term_id": "GO:0005886",
  "gene_name": "Contactin-6",
  "gene": "UniProtKB:Q9UQ52",
  "gene_symbol": "CNTN6"
}